{
  "term_id": "GO:0031965",
  "gene_symbol": "OSBPL3",
  "gene": "UniProtKB:Q9H4L5",
  "gene_name": "Oxysterol-binding protein-related protein 3",
  "term_label": "nuclear membrane"
}